{
  "gene_symbol": "HOXD9",
  "term_id": "GO:0009954",
  "term_label": "proximal/distal pattern formation",
  "gene_name": "Homeobox protein Hox-D9",
  "gene": "UniProtKB:P28356"
}